{
  "gene": "UniProtKB:P12814",
  "gene_name": "Alpha-actinin-1",
  "term_id": "GO:0005886",
  "gene_symbol": "ACTN1",
  "term_label": "plasma membrane"
}